{
  "gene": "UniProtKB:Q9NV64",
  "gene_name": "Transmembrane protein 39A",
  "term_id": "UNKNOWN:0001",
  "term_label": "Unknown molecular function",
  "gene_symbol": "TMEM39A"
}